{
  "gene_name": "Vesicle transport protein SFT2A",
  "gene_symbol": "SFT2D1",
  "term_label": "Unknown biological process",
  "term_id": "UNKNOWN:0002",
  "gene": "UniProtKB:Q8WV19"
}